{
  "term_id": "GO:0005886",
  "gene_name": "Protocadherin-19",
  "gene": "UniProtKB:Q8TAB3",
  "term_label": "plasma membrane",
  "gene_symbol": "PCDH19"
}